pigment metabolic process involved in developmental pigmentation [GO:0043324] (BP) Subtypes: eye pigment metabolic process [GO:0042441], pigment biosynthetic process involved in pigment granule maturation [GO:0048784] Also known as: pigment metabolic process during developmental pigmentation, pigment metabolism during developmental pigmentation Sources: GOC:jl, ISBN:0198506732 Relationships: is a type of pigment metabolic process involved in pigmentation [GO:0043474]; is part of developmental pigmentation [GO:0048066] Definition: The chemical reactions and pathways involving biological pigments e.g. melanin, occurring as part of the development of an organ or organism.